regulation of spore-bearing organ development [GO:0075260] (biological process) Sources: GOC:pamgo_curators Definition: Any process that modulates the frequency, rate or extent of spore-bearing organ development, a process in which hyphae grow into special aggregates called fruiting bodies that produce new spores. Relationships: is a type of regulation of developmental process [GO:0050793]; is a type of regulation of reproductive process [GO:2000241]; regulates GO:0075259 Subtypes: regulation of reproductive fruiting body development [GO:0031155], regulation of conidiophore development [GO:0070793], positive regulation of spore-bearing organ development [GO:0075261], GO:0075262, regulation of oogonium development [GO:0075264], GO:0075272, regulation of telium development [GO:0075276], regulation of uredinium development [GO:0075280], regulation of sporangium development [GO:0075310], regulation of basidium development [GO:0075314], regulation of ascus development [GO:0075318]